{
  "gene_symbol": "SLC25A3",
  "term_label": "phosphate ion transmembrane transport",
  "term_id": "GO:0035435",
  "gene": "UniProtKB:Q00325",
  "gene_name": "Solute carrier family 25 member 3"
}